adenohypophysis development [GO:0021984] (biological process) Also known as: adenophysis development, anterior pituitary development, anterior pituitary gland development Relationships: is a type of GO:0048856; is part of pituitary gland development [GO:0021983] Sources: GOC:cls, GOC:dgh, GOC:dph, GOC:jid, GO_REF:0000021 Definition: The progression of the adenohypophysis over time from its initial formation until its mature state. The adenohypophysis is the anterior part of the pituitary. It secretes a variety of hormones and its function is regulated by the hypothalamus.